{
  "gene_symbol": "GOT1L1",
  "gene": "UniProtKB:Q8NHS2",
  "gene_name": "Putative aspartate aminotransferase, cytoplasmic 2",
  "term_label": "L-aspartate:2-oxoglutarate aminotransferase activity",
  "term_id": "GO:0004069"
}